{
  "gene_name": "Autophagy-related protein 16-1",
  "gene_symbol": "ATG16L1",
  "gene": "UniProtKB:Q676U5",
  "term_id": "GO:0000421",
  "term_label": "autophagosome membrane"
}